{
  "gene": "UniProtKB:P20393",
  "gene_name": "Nuclear receptor subfamily 1 group D member 1",
  "gene_symbol": "NR1D1",
  "term_id": "GO:0045944",
  "term_label": "positive regulation of transcription by RNA polymerase II"
}